action potential propagation [GO:0098870] (biological process) Subtypes: neuronal action potential propagation [GO:0019227], neuronal action potential back-propagation [GO:0098873] Relationships: is a type of action potential [GO:0001508] Sources: GOC:dos Definition: The propagation of an action potential along the plane of an excitable membrane. Action potentials typically propagate once triggered because the depolarization of adjacent membrane regions due to an action potential crosses the firing threshold.